{
  "gene": "UniProtKB:P02741",
  "gene_symbol": "CRP",
  "gene_name": "C-reactive protein",
  "term_label": "innate immune response",
  "term_id": "GO:0045087"
}